squamous basal epithelial stem cell differentiation involved in prostate gland acinus development [GO:0060529] (biological process) References: PMID:18977204 Sources: GOC:dph Relationships: is a type of GO:0002067; is_a stem cell differentiation [GO:0048863]; is a type of epithelial cell differentiation involved in prostate gland development [GO:0060742]; is part of prostate glandular acinus development [GO:0060525] Definition: The process in which a relatively unspecialized epithelial cell acquires specialized features of a squamous basal epithelial stem cell of the prostate.